{
  "term_label": "lysosome",
  "gene_name": "AP-5 complex subunit mu-1",
  "gene": "UniProtKB:Q9H0R1",
  "gene_symbol": "AP5M1",
  "term_id": "GO:0005764"
}